{
  "term_id": "UNKNOWN:0002",
  "gene_name": "G patch domain and ankyrin repeat-containing protein 1",
  "gene_symbol": "GPANK1",
  "gene": "UniProtKB:O95872",
  "term_label": "Unknown biological process"
}